{
  "gene": "UniProtKB:A0A0B4J1X5",
  "gene_symbol": "IGHV3-74",
  "gene_name": "Immunoglobulin heavy variable 3-74",
  "term_label": "immunoglobulin mediated immune response",
  "term_id": "GO:0016064"
}